{
  "term_id": "GO:0043025",
  "term_label": "neuronal cell body",
  "gene_name": "Beta-synuclein",
  "gene_symbol": "SNCB",
  "gene": "UniProtKB:Q16143"
}